{
  "gene": "UniProtKB:Q53EP0",
  "term_label": "Unknown biological process",
  "gene_name": "Fibronectin type III domain-containing protein 3B",
  "term_id": "UNKNOWN:0002",
  "gene_symbol": "FNDC3B"
}